{
  "gene_name": "Putative homeobox protein Meis3-like 1",
  "term_id": "GO:0009880",
  "gene": "UniProtKB:A6NDR6",
  "gene_symbol": "MEIS3P1",
  "term_label": "embryonic pattern specification"
}